{
  "term_label": "Fanconi anaemia nuclear complex",
  "gene_symbol": "FANCB",
  "gene": "UniProtKB:Q8NB91",
  "term_id": "GO:0043240",
  "gene_name": "Fanconi anemia group B protein"
}